nucleolus organization [GO:0007000] (biological process) Also known as: nucleolus organisation, nucleolus organization and biogenesis Sources: GOC:dph, GOC:jid, GOC:jl, GOC:mah Subtypes: nucleologenesis [GO:0017126] Definition: A process that is carried out at the cellular level which results in the assembly, arrangement of constituent parts, or disassembly of the nucleolus. Relationships: is a type of nucleus organization [GO:0006997]